new cell pole [GO:1990902] (cellular component) Definition: The cell pole proximal to the most recent cell division. Relationships: is a type of cell pole [GO:0060187] References: PMID:10231492, PMID:8226658 Sources: GOC:jh2